{
  "gene_name": "Bromodomain-containing protein 3",
  "gene_symbol": "BRD3",
  "term_label": "protein serine/threonine kinase activity",
  "gene": "UniProtKB:Q15059",
  "term_id": "GO:0004674"
}